glycine betaine catabolic process [GO:0031457] (BP) Also known as: N-trimethylglycine catabolic process, N-trimethylglycine catabolism, glycine betaine breakdown, glycine betaine catabolism, glycine betaine degradation Sources: GOC:mah Relationships: is a type of amino-acid betaine catabolic process [GO:0006579] Definition: The chemical reactions and pathways resulting in the breakdown of glycine betaine, N-trimethylglycine.